{
  "term_label": "nuclear steroid receptor activity",
  "gene_symbol": "PAQR7",
  "gene": "UniProtKB:Q86WK9",
  "gene_name": "Membrane progestin receptor alpha",
  "term_id": "GO:0003707"
}